gibberellin 2-beta-dioxygenase activity [GO:0045543] (molecular function) Definition: Catalysis of the reaction: a gibberellin + 2-oxoglutarate + O2 = a 2-beta-hydroxygibberellin + succinate + CO2. References: PMID:32652020 Sources: EC:1.14.11.13 Also known as: gibberellin 2-oxidase activity, gibberellin 2-beta-hydroxylase activity, gibberellin 2beta-dioxygenase activity, gibberellin 2beta-hydroxylase activity Relationships: is a type of 2-oxoglutarate-dependent dioxygenase activity [GO:0016706]